{
  "gene_symbol": "AKAP10",
  "term_id": "UNKNOWN:0001",
  "gene": "UniProtKB:O43572",
  "gene_name": "A-kinase anchor protein 10, mitochondrial",
  "term_label": "Unknown molecular function"
}